{
  "gene_symbol": "FBXO31",
  "term_label": "SCF-dependent proteasomal ubiquitin-dependent protein catabolic process",
  "gene": "UniProtKB:Q5XUX0",
  "term_id": "GO:0031146",
  "gene_name": "F-box only protein 31"
}